{
  "term_id": "GO:0031201",
  "gene": "UniProtKB:Q9BV40",
  "term_label": "SNARE complex",
  "gene_name": "Vesicle-associated membrane protein 8",
  "gene_symbol": "VAMP8"
}